{
  "gene": "UniProtKB:P86434",
  "gene_symbol": "ADORA2A-AS1",
  "term_id": "UNKNOWN:0003",
  "gene_name": "Putative uncharacterized protein ADORA2A-AS1",
  "term_label": "Unknown cellular component"
}